regulation of B-1 B cell differentiation [GO:0001924] (biological process) Definition: Any process that modulates the frequency, rate, or extent of B-1 B cell differentiation. B-1 B cells are a distinct subset of B cells characterized as being CD5 positive, found predominantly in the peritoneum, pleural cavities, and spleen, and enriched for self-reactivity. Subtypes: negative regulation of B-1 B cell differentiation [GO:0001925], positive regulation of B-1 B cell differentiation [GO:0001926] Sources: GOC:add, ISBN:0781735149 Also known as: regulation of B-1 B lymphocyte differentiation, regulation of B-1 B-cell differentiation, regulation of B-1 B-lymphocyte differentiation, regulation of B-1 B cell development Relationships: is a type of GO:0045577; regulates B-1 B cell differentiation [GO:0001923] Note: Note that immunologists typically use the word 'development' to refer to cells of B or T cell lineages undergoing the process that GO describes as 'cell differentiation'.